{
  "gene": "UniProtKB:P21860",
  "gene_name": "Receptor tyrosine-protein kinase erbB-3",
  "term_label": "neuregulin binding",
  "gene_symbol": "ERBB3",
  "term_id": "GO:0038132"
}